{
  "term_label": "plasma membrane",
  "gene_name": "Claudin-7",
  "term_id": "GO:0005886",
  "gene_symbol": "CLDN7",
  "gene": "UniProtKB:O95471"
}